{
  "gene_symbol": "GM2A",
  "gene_name": "Ganglioside GM2 activator",
  "term_id": "GO:0006869",
  "term_label": "lipid transport",
  "gene": "UniProtKB:P17900"
}